{
  "gene_name": "Zinc finger protein 442",
  "term_label": "RNA polymerase II transcription regulatory region sequence-specific DNA binding",
  "term_id": "GO:0000977",
  "gene_symbol": "ZNF442",
  "gene": "UniProtKB:Q9H7R0"
}